negative regulation of vacuole fusion, non-autophagic [GO:0061192] (BP) Relationships: is a type of negative regulation of organelle organization [GO:0010639]; is a type of GO:0032889; RO_0002212 vacuole fusion, non-autophagic [GO:0042144] Definition: Any process that decreases the frequency, rate or extent of the fusion of two vacuole membranes to form a single vacuole. Sources: GOC:dph